{
  "gene": "UniProtKB:O00329",
  "gene_symbol": "PIK3CD",
  "term_label": "phosphatidylinositol-mediated signaling",
  "gene_name": "Phosphatidylinositol 4,5-bisphosphate 3-kinase catalytic subunit delta isoform",
  "term_id": "GO:0048015"
}